{
  "term_id": "GO:0098973",
  "term_label": "structural constituent of postsynaptic actin cytoskeleton",
  "gene_name": "Putative beta-actin-like protein 3",
  "gene": "UniProtKB:Q9BYX7",
  "gene_symbol": "POTEKP"
}